{
  "term_label": "enzyme binding",
  "gene_name": "UDP-glucuronosyltransferase 1A1",
  "gene_symbol": "UGT1A1",
  "gene": "UniProtKB:P22309",
  "term_id": "GO:0019899"
}